{
  "term_label": "neuron projection",
  "term_id": "GO:0043005",
  "gene_name": "Regulator of G-protein signaling 9",
  "gene": "UniProtKB:O75916",
  "gene_symbol": "RGS9"
}